{
  "term_id": "GO:0051754",
  "gene": "UniProtKB:P30154",
  "gene_name": "Serine_threonine-protein phosphatase 2A 65 kDa regulatory subunit A beta isoform",
  "gene_symbol": "PPP2R1B",
  "term_label": "meiotic sister chromatid cohesion, centromeric"
}